cell-cell adhesion mediated by integrin [GO:0033631] (biological process) Regulation: regulated by GO:0033632; negatively regulated by negative regulation of cell-cell adhesion mediated by integrin [GO:0033633]; RO_0002213 by GO:0033634 Also known as: cell-cell adhesion mediated by integrin complex References: PMID:12213832, PMID:14754902 Sources: GOC:add Relationships: is a type of cell adhesion mediated by integrin [GO:0033627]; is_a GO:0098609 Definition: The attachment of one cell to another cell via an integrin, a heterodimeric adhesion receptor formed by the non-covalent association of particular alpha and beta subunits.